{
  "gene_symbol": "OR4E2",
  "term_label": "detection of chemical stimulus involved in sensory perception of smell",
  "gene_name": "Olfactory receptor 4E2",
  "gene": "UniProtKB:Q8NGC2",
  "term_id": "GO:0050911"
}